{
  "gene": "UniProtKB:Q8NAN2",
  "term_id": "UNKNOWN:0001",
  "term_label": "Unknown molecular function",
  "gene_name": "Mitoguardin 1",
  "gene_symbol": "MIGA1"
}